regulation of T-helper 2 cell activation [GO:2000569] (biological process) Definition: Any process that modulates the frequency, rate or extent of T-helper 2 cell activation. Sources: GOC:obol Also known as: regulation of Th2 cell activation Subtypes: positive regulation of T-helper 2 cell activation [GO:2000570] Relationships: is a type of regulation of CD4-positive, alpha-beta T cell activation [GO:2000514]; regulates T-helper 2 cell activation [GO:0035712]